{
  "gene_name": "Serologically defined colon cancer antigen 8",
  "gene_symbol": "SDCCAG8",
  "term_label": "neuron migration",
  "term_id": "GO:0001764",
  "gene": "UniProtKB:Q86SQ7"
}